{
  "gene_symbol": "MSL1",
  "term_id": "GO:0003682",
  "gene": "UniProtKB:Q68DK7",
  "term_label": "chromatin binding",
  "gene_name": "Male-specific lethal 1 homolog"
}